{
  "gene": "UniProtKB:Q9Y4X3",
  "term_label": "antimicrobial humoral immune response mediated by antimicrobial peptide",
  "gene_name": "C-C motif chemokine 27",
  "term_id": "GO:0061844",
  "gene_symbol": "CCL27"
}